{
  "term_id": "GO:0060271",
  "gene": "UniProtKB:Q9Y592",
  "term_label": "cilium assembly",
  "gene_name": "Centrosomal protein of 83 kDa",
  "gene_symbol": "CEP83"
}